regulation of mRNA processing [GO:0050684] (biological process) Definition: Any process that modulates the frequency, rate or extent of mRNA processing, those processes involved in the conversion of a primary mRNA transcript into a mature mRNA prior to its translation into polypeptide. Sources: GOC:ai Relationships: is_a regulation of mRNA metabolic process [GO:1903311]; regulates mRNA processing [GO:0006397] Subtypes: regulation of mRNA 3'-end processing [GO:0031440], regulation of mRNA splicing, via spliceosome [GO:0048024], positive regulation of mRNA processing [GO:0050685], negative regulation of mRNA processing [GO:0050686]